{
  "term_id": "GO:0008013",
  "gene": "UniProtKB:Q9UKB5",
  "term_label": "beta-catenin binding",
  "gene_symbol": "AJAP1",
  "gene_name": "Adherens junction-associated protein 1"
}